actin wave [GO:0062201] (cellular component) References: PMID:26190109, PMID:31230946, PMID:31390543, PMID:31678045, PMID:31774725 Definition: A cellular anatomical entity that is part of the actin cytoskeleton and results in a wave-like propagation of actin networks. It consists of dynamic structures traveling on the ventral (substrate-attached) side of the cell during cell migration, cytokinesis, adhesion and neurogenesis. Relationships: is a type of cellular anatomical structure [GO:0110165]; is part of actin cytoskeleton [GO:0015629]; has part actin filament [GO:0005884]